{
  "gene_name": "Secretogranin-1",
  "term_id": "GO:0030141",
  "term_label": "secretory granule",
  "gene": "UniProtKB:P05060",
  "gene_symbol": "CHGB"
}